ITP diphosphatase activity [GO:0036220] (molecular function) References: PMID:17899088, PMID:22531138 Sources: GOC:dgf, RHEA:29399 Also known as: ITP pyrophosphatase activity, inosine-5'-triphosphate pyrophosphohydrolase activity Definition: Catalysis of the reaction: ITP + H2O = IMP + H+ + diphosphate. Relationships: is a type of GO:0047429